{
  "term_label": "regulation of transcription by RNA polymerase II",
  "gene": "UniProtKB:Q9NU39",
  "gene_name": "Forkhead box protein D4-like 1",
  "term_id": "GO:0006357",
  "gene_symbol": "FOXD4L1"
}